{
  "gene": "UniProtKB:O95487",
  "gene_name": "Protein transport protein Sec24B",
  "term_label": "zinc ion binding",
  "gene_symbol": "SEC24B",
  "term_id": "GO:0008270"
}